{
  "term_id": "GO:0005922",
  "gene": "UniProtKB:Q8N144",
  "term_label": "connexin complex",
  "gene_symbol": "GJD3",
  "gene_name": "Gap junction delta-3 protein"
}